{
  "term_label": "nucleus",
  "gene": "UniProtKB:P80294",
  "term_id": "GO:0005634",
  "gene_symbol": "MT1H",
  "gene_name": "Metallothionein-1H"
}